chromoplast inner membrane [GO:0031899] (cellular component) Definition: The inner, i.e. lumen-facing, lipid bilayer of the chromoplast envelope; also faces the chromoplast stroma. Relationships: is a type of GO:0009528; is a type of GO:0046862 Sources: GOC:pz